{
  "term_id": "GO:0004674",
  "gene_symbol": "NEK9",
  "gene": "UniProtKB:Q8TD19",
  "term_label": "protein serine/threonine kinase activity",
  "gene_name": "Serine_threonine-protein kinase Nek9"
}